{
  "gene_symbol": "GSDMB",
  "term_label": "pyroptotic inflammatory response",
  "gene": "UniProtKB:Q8TAX9",
  "gene_name": "Gasdermin-B",
  "term_id": "GO:0070269"
}